{
  "gene_name": "Carcinoembryonic antigen-related cell adhesion molecule 16",
  "term_label": "Unknown molecular function",
  "term_id": "UNKNOWN:0001",
  "gene": "UniProtKB:Q2WEN9",
  "gene_symbol": "CEACAM16"
}